{
  "gene": "UniProtKB:Q9Y2Q3",
  "term_label": "peroxisome",
  "gene_name": "Glutathione S-transferase kappa 1",
  "term_id": "GO:0005777",
  "gene_symbol": "GSTK1"
}